{
  "gene_name": "WAP four-disulfide core domain protein 5",
  "term_label": "innate immune response",
  "term_id": "GO:0045087",
  "gene_symbol": "WFDC5",
  "gene": "UniProtKB:Q8TCV5"
}